{
  "gene": "UniProtKB:Q14191",
  "term_label": "nucleoplasm",
  "term_id": "GO:0005654",
  "gene_symbol": "WRN",
  "gene_name": "Bifunctional 3'-5' exonuclease_ATP-dependent helicase WRN"
}